glycogen cell differentiation involved in embryonic placenta development [GO:0060709] (biological process) Relationships: is a type of cell differentiation involved in embryonic placenta development [GO:0060706]; is part of spongiotrophoblast layer development [GO:0060712] References: PMID:16269175 Sources: GOC:dph Definition: The process in which a relatively unspecialized cell acquires specialized features of a glycogen cell of the placenta. A glycogen cell is a vacuolated glycogen-rich cell that appears in compact cell islets of the spongiotrophoblast layer.